{
  "gene_symbol": "C5AR2",
  "term_id": "GO:0016323",
  "gene_name": "C5a anaphylatoxin chemotactic receptor 2",
  "term_label": "basolateral plasma membrane",
  "gene": "UniProtKB:Q9P296"
}